meiotic attachment of telomere to nuclear envelope [GO:0070197] (biological process) Definition: The meiotic cell cycle process in which physical connections are formed between telomeric heterochromatin and the nuclear envelope, facilitating bouquet formation. Relationships: is a type of chromosome attachment to the nuclear envelope [GO:0097240]; is a type of meiotic cell cycle process [GO:1903046]; is part of GO:0044821 References: PMID:18818742 Sources: GOC:jp, GOC:pr, GOC:vw Also known as: attachment of telomeres to nuclear envelope, attachment of telomeric chromatin to nuclear envelope